transmitter-gated monoatomic ion channel activity involved in regulation of postsynaptic membrane potential [GO:1904315] (molecular function) Subtypes: acetylcholine-gated monoatomic cation-selective channel activity [GO:0022848] References: PMID:20200227 Sources: GOC:TermGenie, GO_REF:0000061 Also known as: transmitter-gated ion channel activity involved in regulation of postsynaptic membrane potential, ionotropic neurotransmitter receptor activity involved in regulation of post-synaptic membrane potential, ionotropic neurotransmitter receptor activity involved in regulation of postsynaptic membrane potential Definition: Any transmitter-gated ion channel activity that is involved in regulation of postsynaptic membrane potential. Relationships: is a type of transmitter-gated monoatomic ion channel activity [GO:0022824]; is a type of neurotransmitter receptor activity involved in regulation of postsynaptic membrane potential [GO:0099529]